{
  "term_id": "UNKNOWN:0002",
  "term_label": "Unknown biological process",
  "gene_symbol": "RBM22",
  "gene_name": "Pre-mRNA-splicing factor RBM22",
  "gene": "UniProtKB:Q9NW64"
}